{
  "term_label": "Unknown biological process",
  "gene_symbol": "FAM217A",
  "gene_name": "Protein FAM217A",
  "gene": "UniProtKB:Q8IXS0",
  "term_id": "UNKNOWN:0002"
}